{
  "term_label": "mannosyltransferase activity",
  "gene": "UniProtKB:Q9NUD9",
  "gene_name": "GPI mannosyltransferase 2",
  "gene_symbol": "PIGV",
  "term_id": "GO:0000030"
}